positive regulation of (+)-kotanin biosynthetic process [GO:1900694] (biological process) Also known as: activation of (+)-kotanin anabolism, activation of (+)-kotanin biosynthesis, activation of (+)-kotanin formation, activation of (+)-kotanin synthesis, positive regulation of (+)-kotanin anabolism, positive regulation of (+)-kotanin biosynthesis, positive regulation of (+)-kotanin formation, positive regulation of (+)-kotanin synthesis, up regulation of (+)-kotanin anabolism, up regulation of (+)-kotanin biosynthesis, up regulation of (+)-kotanin biosynthetic process, up regulation of (+)-kotanin formation, up regulation of (+)-kotanin synthesis, up-regulation of (+)-kotanin anabolism, up-regulation of (+)-kotanin biosynthesis, up-regulation of (+)-kotanin biosynthetic process, up-regulation of (+)-kotanin formation, up-regulation of (+)-kotanin synthesis, upregulation of (+)-kotanin anabolism, upregulation of (+)-kotanin biosynthesis, upregulation of (+)-kotanin biosynthetic process, upregulation of (+)-kotanin formation, upregulation of (+)-kotanin synthesis, activation of (+)-kotanin biosynthetic process Definition: Any process that activates or increases the frequency, rate or extent of (+)-kotanin biosynthetic process. Sources: GOC:TermGenie, GOC:di Relationships: is a type of positive regulation of secondary metabolite biosynthetic process [GO:1900378]; is a type of regulation of (+)-kotanin biosynthetic process [GO:1900692]; positively regulates (+)-kotanin biosynthetic process [GO:1900596]